{
  "term_id": "UNKNOWN:0002",
  "gene": "UniProtKB:A0A075B6W6",
  "gene_name": "T cell receptor alpha joining 27 (Fragment)",
  "gene_symbol": "TRAJ27",
  "term_label": "Unknown biological process"
}